{
  "term_id": "GO:0035249",
  "gene_name": "Glutamate receptor ionotropic, NMDA 2C",
  "gene": "UniProtKB:Q14957",
  "gene_symbol": "GRIN2C",
  "term_label": "synaptic transmission, glutamatergic"
}